{
  "gene_name": "HLA class II histocompatibility antigen, DR beta 3 chain",
  "term_id": "GO:0050778",
  "term_label": "positive regulation of immune response",
  "gene_symbol": "HLA-DRB3",
  "gene": "UniProtKB:P79483"
}